protein C inhibitor-PLAT complex [GO:0036026] (cellular component) Relationships: is a type of serine protease inhibitor complex [GO:0097180] Definition: A heterodimeric protein complex that contains protein C inhibitor (SERPINA5) and tissue-type plasminogen activator (PLAT); formation of the complex inhibits the serine protease activity of tissue-type plasminogen activator. References: PMID:10340997 Sources: GOC:ans Also known as: PCI-PLAT complex, SERPINA5-PLAT complex, plasma serine protease inhibitor-PLAT complex, protein C inhibitor-tPA complex, protein C inhibitor-tissue-type plasminogen activator complex, serpin A5-PLAT complex